negative regulation of xenophagy [GO:1904416] (biological process) Relationships: is a type of negative regulation of response to biotic stimulus [GO:0002832]; is a type of negative regulation of macroautophagy [GO:0016242]; is a type of negative regulation of defense response [GO:0031348]; is a type of negative regulation of response to external stimulus [GO:0032102]; is a type of GO:1904415; negatively regulates xenophagy [GO:0098792] Also known as: down regulation of xenophagy, down-regulation of xenophagy, downregulation of xenophagy, inhibition of xenophagy References: PMID:21617041 Sources: GOC:PARL, GOC:TermGenie, GOC:pad, GO_REF:0000058 Definition: Any process that stops, prevents or reduces the frequency, rate or extent of xenophagy. Note: An example of this is mouse Tbk1 (UniProt symbol, Q9WUN2) in PMID:21617041 (inferred from mutant phenotype).